{
  "term_label": "mitochondrial electron transport, NADH to ubiquinone",
  "term_id": "GO:0006120",
  "gene": "UniProtKB:P03891",
  "gene_symbol": "MT-ND2",
  "gene_name": "NADH-ubiquinone oxidoreductase chain 2"
}